{
  "term_id": "GO:0005634",
  "gene_symbol": "CSNK1A1",
  "gene": "UniProtKB:P48729",
  "gene_name": "Casein kinase I isoform alpha",
  "term_label": "nucleus"
}